anterior midgut (ectodermal) morphogenesis [GO:0007441] (biological process) Sources: GOC:go_curators Relationships: is_a GO:0002009; is part of ectodermal digestive tract morphogenesis [GO:0048567] Definition: The process in which the anatomical structures of the anterior midgut (ectodermal) are generated and organized.